{
  "term_label": "Unknown biological process",
  "gene_symbol": "SMIM43",
  "term_id": "UNKNOWN:0002",
  "gene_name": "Small integral membrane protein 43",
  "gene": "UniProtKB:Q4W5P6"
}